{
  "gene": "UniProtKB:Q495B1",
  "gene_name": "Ankyrin repeat and death domain-containing protein 1A",
  "term_id": "UNKNOWN:0002",
  "term_label": "Unknown biological process",
  "gene_symbol": "ANKDD1A"
}